nitrotoluene catabolic process [GO:0046263] (BP) Sources: GOC:ai Relationships: is a type of toluene-containing compound catabolic process [GO:0072491] Subtypes: 4-nitrotoluene catabolic process [GO:0019258], trinitrotoluene catabolic process [GO:0046260] Also known as: nitrotoluene breakdown, nitrotoluene catabolism, nitrotoluene degradation Definition: The chemical reactions and pathways resulting in the breakdown of nitrotoluene, any methylbenzene molecule with NO2 group(s) attached.